response to epidermal growth factor [GO:0070849] (biological process) Also known as: response to EGF stimulus, response to epidermal growth factor stimulus Subtypes: cellular response to epidermal growth factor stimulus [GO:0071364] Definition: Any process that results in a change in state or activity of a cell or an organism (in terms of movement, secretion, enzyme production, gene expression, etc.) as a result of an epidermal growth factor stimulus. Relationships: is a type of response to growth factor [GO:0070848] Sources: GOC:BHF, GOC:mah